{
  "gene_name": "Harmonin",
  "gene_symbol": "USH1C",
  "term_id": "GO:0046549",
  "gene": "UniProtKB:Q9Y6N9",
  "term_label": "retinal cone cell development"
}